{
  "term_label": "Unknown biological process",
  "gene": "UniProtKB:A0A087WU04",
  "term_id": "UNKNOWN:0002",
  "gene_symbol": "TRAJ36",
  "gene_name": "T cell receptor alpha joining 36 (Fragment)"
}